{
  "gene_symbol": "PAPPA2",
  "gene_name": "Pappalysin-2",
  "gene": "UniProtKB:Q9BXP8",
  "term_id": "GO:0005615",
  "term_label": "extracellular space"
}